{
  "gene": "UniProtKB:P49238",
  "gene_symbol": "CX3CR1",
  "term_id": "GO:0006955",
  "term_label": "immune response",
  "gene_name": "CX3C chemokine receptor 1"
}